inositol phosphate biosynthetic process [GO:0032958] (biological process) Sources: GOC:mah Also known as: inositol phosphate anabolism, inositol phosphate biosynthesis, inositol phosphate formation, inositol phosphate synthesis, myo-inositol phosphate biosynthetic process Subtypes: myo-inositol hexakisphosphate biosynthetic process [GO:0010264], inositol trisphosphate biosynthetic process [GO:0032959] Definition: The chemical reactions and pathways resulting in the formation of an inositol phosphate, 1,2,3,4,5,6-cyclohexanehexol, with one or more phosphate groups attached. Regulation: regulated by GO:0010919; negatively regulated by negative regulation of inositol phosphate biosynthetic process [GO:0010920]; positively regulated by positive regulation of inositol phosphate biosynthetic process [GO:0060732] Relationships: is a type of inositol phosphate metabolic process [GO:0043647]; is a type of polyol biosynthetic process [GO:0046173]; is a type of organophosphate biosynthetic process [GO:0090407]